{
  "term_label": "ionotropic glutamate receptor binding",
  "term_id": "GO:0035255",
  "gene_symbol": "NETO1",
  "gene_name": "Neuropilin and tolloid-like protein 1",
  "gene": "UniProtKB:Q8TDF5"
}